{
  "gene": "UniProtKB:O15151",
  "term_id": "GO:0045892",
  "gene_symbol": "MDM4",
  "gene_name": "Protein Mdm4",
  "term_label": "negative regulation of DNA-templated transcription"
}